{
  "term_label": "Unknown molecular function",
  "gene": "UniProtKB:Q9ULC4",
  "gene_name": "Malignant T-cell-amplified sequence 1",
  "term_id": "UNKNOWN:0001",
  "gene_symbol": "MCTS1"
}